cytoophidium organization [GO:0140904] (biological process) Definition: A process which results in the assembly, arrangement of constituent parts, or disassembly of a cytoophidium. Cytoophidia are mesoscale, intracellular, filamentous structures that contain metabolic enzymes. References: PMID:25223282, PMID:27362644 Relationships: is a type of supramolecular fiber organization [GO:0097435]